{
  "gene": "UniProtKB:O95571",
  "term_label": "glutathione metabolic process",
  "term_id": "GO:0006749",
  "gene_name": "Persulfide dioxygenase ETHE1, mitochondrial",
  "gene_symbol": "ETHE1"
}